{
  "gene_symbol": "HAT1",
  "term_id": "UNKNOWN:0003",
  "term_label": "Unknown cellular component",
  "gene_name": "Histone acetyltransferase type B catalytic subunit",
  "gene": "UniProtKB:O14929"
}